negative regulation of membrane tubulation [GO:1903526] (BP) Also known as: down regulation of membrane tubulation, down regulation of plasma membrane tubulation, down-regulation of membrane tubulation, down-regulation of plasma membrane tubulation, downregulation of membrane tubulation, downregulation of plasma membrane tubulation, negative regulation of plasma membrane tubulation, inhibition of membrane tubulation, inhibition of plasma membrane tubulation Definition: Any process that stops, prevents or reduces the frequency, rate or extent of membrane tubulation. Relationships: is a type of GO:0051129; is a type of GO:1903525; negatively regulates plasma membrane tubulation [GO:0097320] References: PMID:18388313 Sources: GOC:TermGenie, GOC:pm, GO_REF:0000058